positive regulation of secretion [GO:0051047] (biological process) Sources: GOC:ai Definition: Any process that activates or increases the frequency, rate or extent of the controlled release of a substance from a cell or a tissue. Relationships: is a type of regulation of secretion [GO:0051046]; is a type of positive regulation of transport [GO:0051050]; positively regulates secretion [GO:0046903] Also known as: up regulation of secretion, up-regulation of secretion, upregulation of secretion, activation of secretion, stimulation of secretion Subtypes: positive regulation of peptide secretion [GO:0002793], positive regulation of gamma-aminobutyric acid secretion [GO:0014054], positive regulation of icosanoid secretion [GO:0032305], positive regulation of renal sodium excretion [GO:0035815], GO:0046878, positive regulation of gastric acid secretion [GO:0060454], positive regulation of mucus secretion [GO:0070257], positive regulation of pancreatic juice secretion [GO:0090187], GO:0120189, positive regulation of lactation [GO:1903489], GO:1903532, positive regulation of defecation [GO:2000294]